{
  "gene_name": "Triple QxxK_R motif-containing protein",
  "term_id": "UNKNOWN:0003",
  "gene_symbol": "TRIQK",
  "gene": "UniProtKB:Q629K1",
  "term_label": "Unknown cellular component"
}